{
  "term_id": "UNKNOWN:0003",
  "term_label": "Unknown cellular component",
  "gene_symbol": "CXorf58",
  "gene": "UniProtKB:Q96LI9",
  "gene_name": "Uncharacterized protein CXorf58"
}